{
  "gene": "UniProtKB:Q8IYR2",
  "gene_name": "SET and MYND domain-containing protein 4",
  "term_id": "GO:0042826",
  "gene_symbol": "SMYD4",
  "term_label": "histone deacetylase binding"
}